{
  "gene_name": "Putative protein ZNF321",
  "term_label": "Unknown biological process",
  "gene": "UniProtKB:Q8N8H1",
  "term_id": "UNKNOWN:0002",
  "gene_symbol": "ZNF321P"
}